Casparian strip [GO:0048226] (cellular component) Sources: GOC:jid Relationships: is a type of cellular anatomical structure [GO:0110165]; is part of GO:0009531 Definition: Region of plant cell wall specialised to act as a seal to prevent back leakage of secreted material (analogous to tight junction between epithelial cells). Found particularly where root parenchymal cells secrete solutes into xylem vessels. The barrier is composed of suberin; a fatty substance, containing long chain fatty acids and fatty esters, also found in the cell walls of cork cells (phellem) in higher plants.